{
  "gene": "UniProtKB:Q9H0A9",
  "gene_name": "Speriolin-like protein",
  "term_id": "GO:0034237",
  "term_label": "protein kinase A regulatory subunit binding",
  "gene_symbol": "SPATC1L"
}